{
  "term_id": "GO:0016887",
  "term_label": "ATP hydrolysis activity",
  "gene": "UniProtKB:O43896",
  "gene_name": "Kinesin-like protein KIF1C",
  "gene_symbol": "KIF1C"
}